eNoSc complex [GO:0061773] (cellular component) Relationships: is a type of chromatin silencing complex [GO:0005677]; is part of GO:0005730 Definition: A chromatin silencing complex that recruits histone-modifying enzymes and upregulates silencing of rDNA in response to glucose starvation. Also known as: energy dependent nucleolar silencing complex References: PMID:18485871 Sources: GOC:BHM